{
  "gene_name": "Solute carrier family 2, facilitated glucose transporter member 14",
  "term_id": "GO:0070837",
  "gene_symbol": "SLC2A14",
  "term_label": "dehydroascorbic acid transport",
  "gene": "UniProtKB:Q8TDB8"
}